{
  "gene_name": "DAZ-associated protein 1",
  "term_label": "mRNA 3'-UTR binding",
  "gene": "UniProtKB:Q96EP5",
  "gene_symbol": "DAZAP1",
  "term_id": "GO:0003730"
}